{
  "gene": "UniProtKB:Q13576",
  "term_id": "GO:0005938",
  "gene_symbol": "IQGAP2",
  "term_label": "cell cortex",
  "gene_name": "Ras GTPase-activating-like protein IQGAP2"
}